regulation of blood volume by renal aldosterone [GO:0002017] (biological process) Relationships: is a type of renal system process involved in regulation of blood volume [GO:0001977]; is a type of regulation of systemic arterial blood pressure by hormone [GO:0001990]; is a type of GO:0003084 Sources: GOC:dph, GOC:tb, ISBN:0721643949 Definition: The process in which the hormone aldosterone decreases the rate of diuresis and natriuresis resulting in increased blood volume. Also known as: aldosterone mediated regulation of blood volume, renal regulation of blood volume by aldosterone, aldosterone mediated control of body fluids